{
  "term_label": "chromosome segregation",
  "term_id": "GO:0007059",
  "gene_name": "Centromere protein W",
  "gene_symbol": "CENPW",
  "gene": "UniProtKB:Q5EE01"
}